{
  "gene_name": "Protein EURL homolog",
  "term_label": "Unknown biological process",
  "gene": "UniProtKB:Q9NYK6",
  "gene_symbol": "EURL",
  "term_id": "UNKNOWN:0002"
}